{
  "term_label": "Unknown biological process",
  "gene_symbol": "CRCT1",
  "gene_name": "Cysteine-rich C-terminal protein 1",
  "term_id": "UNKNOWN:0002",
  "gene": "UniProtKB:Q9UGL9"
}